{
  "term_label": "establishment or maintenance of cell polarity",
  "term_id": "GO:0007163",
  "gene_name": "Ras-related protein R-Ras2",
  "gene_symbol": "RRAS2",
  "gene": "UniProtKB:P62070"
}